{
  "term_id": "UNKNOWN:0001",
  "gene": "UniProtKB:Q969F2",
  "gene_symbol": "NKD2",
  "gene_name": "Protein naked cuticle homolog 2",
  "term_label": "Unknown molecular function"
}